{
  "term_label": "adherens junction",
  "term_id": "GO:0005912",
  "gene": "UniProtKB:Q9NR12",
  "gene_symbol": "PDLIM7",
  "gene_name": "PDZ and LIM domain protein 7"
}